{
  "gene": "UniProtKB:Q14185",
  "term_label": "cell migration",
  "gene_name": "Dedicator of cytokinesis protein 1",
  "gene_symbol": "DOCK1",
  "term_id": "GO:0016477"
}